{
  "gene_name": "Large ribosomal subunit protein mL53",
  "term_label": "mitochondrial large ribosomal subunit",
  "gene_symbol": "MRPL53",
  "gene": "UniProtKB:Q96EL3",
  "term_id": "GO:0005762"
}